dTDP-glucose 4,6-dehydratase activity [GO:0008460] (molecular function) Also known as: TDP-glucose oxidoreductase activity, dTDP-glucose 4,6-hydro-lyase (dTDP-4-dehydro-6-deoxy-D-glucose-forming), dTDP-glucose 4,6-hydro-lyase activity, dTDPglucose 4,6-dehydratase activity, dTDPglucose 4,6-hydro-lyase activity, thymidine diphosphoglucose oxidoreductase activity Sources: EC:4.2.1.46, RHEA:17221 Relationships: is a type of hydro-lyase activity [GO:0016836] Definition: Catalysis of the reaction: dTDP-glucose = dTDP-4-dehydro-6-deoxy-alpha-D-glucose + H2O.